{
  "term_label": "pre-mRNA 3'-splice site binding",
  "gene_symbol": "ZRSR2P1",
  "term_id": "GO:0030628",
  "gene_name": "Putative U2 small nuclear ribonucleoprotein auxiliary factor 35 kDa subunit-related protein 1",
  "gene": "UniProtKB:Q15695"
}